positive regulation of response to amylopectin [GO:1900523] (biological process) Also known as: up regulation of response to amylopectin, up-regulation of response to amylopectin, upregulation of response to amylopectin, activation of response to amylopectin Definition: Any process that activates or increases the frequency, rate or extent of response to amylopectin. Sources: GOC:TermGenie, GOC:mengo_curators Relationships: is a type of positive regulation of response to stimulus [GO:0048584]; is a type of GO:1900521; positively regulates response to amylopectin [GO:0044591]